regulation of P-type sodium:potassium-exchanging transporter activity [GO:1903406] (biological process) Subtypes: negative regulation of P-type sodium:potassium-exchanging transporter activity [GO:1903407], positive regulation of P-type sodium:potassium-exchanging transporter activity [GO:1903408] Relationships: is a type of GO:0043462; is a type of regulation of sodium ion transmembrane transporter activity [GO:2000649]; regulates GO:0005391 Definition: Any process that modulates the frequency, rate or extent of sodium:potassium-exchanging ATPase activity. Also known as: regulation of sodium pump, regulation of (Na+ + K+)-ATPase activity, regulation of (Na+ + K+)-activated ATPase activity, regulation of ATP phosphohydrolase (Na+/K+-exchanging), regulation of Na(+)/K(+)-ATPase activity, regulation of Na(+)/K(+)-exchanging ATPase activity, regulation of Na+,K+-ATPase activity, regulation of Na+/K+-ATPase activity, regulation of Na+/K+-exchanging ATPase activity, regulation of Na,K-activated ATPase activity, regulation of sodium/potassium-exchanging ATPase activity, regulation of sodium/potassium-transporting ATPase activity, regulation of sodium:potassium exchanging ATPase activity, regulation of sodium:potassium-exchanging ATPase activity, regulation of Na+,K+ pump, regulation of Na,K-pump References: PMID:8160880 Sources: GOC:TermGenie, GOC:mr, GO_REF:0000059